{
  "gene": "UniProtKB:Q5TA45",
  "gene_symbol": "INTS11",
  "gene_name": "Integrator complex subunit 11",
  "term_label": "nucleus",
  "term_id": "GO:0005634"
}